{
  "gene_symbol": "MEIS1",
  "term_id": "GO:0007420",
  "term_label": "brain development",
  "gene": "UniProtKB:O00470",
  "gene_name": "Homeobox protein Meis1"
}